CC-preferring endodeoxyribonuclease activity [GO:0033891] (molecular function) Also known as: 5'-CC-3'-preferring endodeoxyribonuclease activity, Streptomyces glaucescens exocytoplasmic dodeoxyribonuclease activity, Streptomyces glaucescens exocytoplasmic endodeoxyribonuclease activity, Streptomyces glaucescens exocytoplasmic endonuclease activity Definition: Catalysis of the endonucleolytic cleavage to give 5'-phosphooligonucleotide end-products, with a preference for cleavage within the sequence CC. Sources: EC:3.1.21.6 Relationships: is_a DNA endonuclease activity, producing 5'-phosphomonoesters [GO:0016888]